{
  "term_label": "nucleus",
  "term_id": "GO:0005634",
  "gene_symbol": "PTGES3L",
  "gene": "UniProtKB:E9PB15",
  "gene_name": "Putative protein PTGES3L"
}